L-ascorbate peroxidase activity [GO:0016688] (molecular function) Definition: Catalysis of the reaction: L-ascorbate + hydrogen peroxide = dehydroascorbate + 2 H2O. Sources: EC:1.11.1.11 Relationships: is a type of peroxidase activity [GO:0004601] Also known as: L-ascorbate:hydrogen-peroxide oxidoreductase activity, L-ascorbic acid peroxidase activity, L-ascorbic acid-specific peroxidase activity, ascorbate peroxidase activity, ascorbic acid peroxidase activity